{
  "gene_name": "Large ribosomal subunit protein mL62",
  "gene_symbol": "MRPL58",
  "gene": "UniProtKB:Q14197",
  "term_label": "mitochondrial large ribosomal subunit",
  "term_id": "GO:0005762"
}